{
  "gene_name": "Alpha-2-macroglobulin-like protein 1",
  "term_id": "UNKNOWN:0001",
  "gene": "UniProtKB:A8K2U0",
  "term_label": "Unknown molecular function",
  "gene_symbol": "A2ML1"
}